{
  "term_label": "5'-deoxynucleotidase activity",
  "term_id": "GO:0002953",
  "gene_symbol": "HDDC2",
  "gene_name": "5'-deoxynucleotidase HDDC2",
  "gene": "UniProtKB:Q7Z4H3"
}